regulation of DNA recombination [GO:0000018] (biological process) Sources: GOC:go_curators, ISBN:0198506732 Definition: Any process that modulates the frequency, rate or extent of DNA recombination, a DNA metabolic process in which a new genotype is formed by reassortment of genes resulting in gene combinations different from those that were present in the parents. Subtypes: regulation of mitotic recombination [GO:0000019], regulation of reciprocal meiotic recombination [GO:0010520], GO:0010569, GO:0045191, negative regulation of DNA recombination [GO:0045910], positive regulation of DNA recombination [GO:0045911], regulation of DNA recombination at centromere [GO:0061806], regulation of DNA recombination at telomere [GO:0072695], regulation of single-strand break repair via homologous recombination [GO:1903110] Relationships: is a type of regulation of DNA metabolic process [GO:0051052]; regulates DNA recombination [GO:0006310]